{
  "gene_symbol": "NDUFS6",
  "term_label": "respiratory chain complex I",
  "gene": "UniProtKB:O75380",
  "gene_name": "NADH dehydrogenase [ubiquinone] iron-sulfur protein 6, mitochondrial",
  "term_id": "GO:0045271"
}